{
  "gene": "UniProtKB:Q9BQS2",
  "gene_symbol": "SYT15",
  "term_id": "GO:0061891",
  "gene_name": "Synaptotagmin-15",
  "term_label": "calcium ion sensor activity"
}